lipid transporter activity [GO:0005319] (molecular function) Also known as: lipophorin, apolipoprotein Definition: Enables the directed movement of lipids into, out of or within a cell, or between cells. Subtypes: phospholipid transporter activity [GO:0005548], sphingolipid transporter activity [GO:0046624], lipid transfer activity [GO:0120013], intramembrane lipid transporter activity [GO:0140303], lipid transmembrane transporter activity [GO:0170055] Relationships: is a type of transporter activity [GO:0005215]; is part of lipid transport [GO:0006869] Sources: GOC:ai